{
  "gene_name": "tRNA-dihydrouridine(47) synthase [NAD(P)(+)]-like",
  "gene": "UniProtKB:Q96G46",
  "term_id": "GO:0017150",
  "gene_symbol": "DUS3L",
  "term_label": "tRNA dihydrouridine synthase activity"
}